{
  "term_id": "GO:0005886",
  "term_label": "plasma membrane",
  "gene_name": "Sodium_hydrogen exchanger 1",
  "gene_symbol": "SLC9A1",
  "gene": "UniProtKB:P19634"
}